{
  "term_id": "GO:0019901",
  "gene_symbol": "CAMK2N2",
  "gene_name": "Calcium_calmodulin-dependent protein kinase II inhibitor 2",
  "term_label": "protein kinase binding",
  "gene": "UniProtKB:Q96S95"
}